{
  "term_label": "G protein-coupled receptor activity",
  "gene_symbol": "MTNR1B",
  "term_id": "GO:0004930",
  "gene_name": "Melatonin receptor type 1B",
  "gene": "UniProtKB:P49286"
}